verbascose synthase activity [GO:0102830] (molecular function) Definition: Catalysis of the reaction: 2 stachyose = verbascose + raffinose. References: PMID:12060258 Sources: GOC:pz Relationships: is a type of hexosyltransferase activity [GO:0016758]